{
  "term_label": "15-hydroxyprostaglandin dehydrogenase (NAD+) activity",
  "gene_name": "15-hydroxyprostaglandin dehydrogenase [NAD(+)]",
  "gene": "UniProtKB:P15428",
  "term_id": "GO:0016404",
  "gene_symbol": "HPGD"
}